{
  "term_id": "GO:0010757",
  "gene": "UniProtKB:P07093",
  "gene_name": "Glia-derived nexin",
  "term_label": "negative regulation of plasminogen activation",
  "gene_symbol": "SERPINE2"
}